{
  "gene_name": "Ubiquitin-conjugating enzyme E2 N",
  "term_id": "GO:0006301",
  "gene_symbol": "UBE2N",
  "term_label": "DNA damage tolerance",
  "gene": "UniProtKB:P61088"
}